{
  "term_id": "GO:0005737",
  "term_label": "cytoplasm",
  "gene": "UniProtKB:P23677",
  "gene_name": "Inositol-trisphosphate 3-kinase A",
  "gene_symbol": "ITPKA"
}